{
  "gene": "UniProtKB:Q14155",
  "term_id": "GO:0005085",
  "gene_name": "Rho guanine nucleotide exchange factor 7",
  "term_label": "guanyl-nucleotide exchange factor activity",
  "gene_symbol": "ARHGEF7"
}